{
  "gene_symbol": "ZNF30",
  "term_id": "GO:0006357",
  "term_label": "regulation of transcription by RNA polymerase II",
  "gene_name": "Zinc finger protein 30",
  "gene": "UniProtKB:P17039"
}